{
  "gene_name": "Putative SAGE1-like protein",
  "gene": "UniProtKB:A6NJ88",
  "term_label": "protein-macromolecule adaptor activity",
  "gene_symbol": "SAGE2P",
  "term_id": "GO:0030674"
}